{
  "gene": "UniProtKB:O75821",
  "term_label": "Unknown molecular function",
  "term_id": "UNKNOWN:0001",
  "gene_symbol": "EIF3G",
  "gene_name": "Eukaryotic translation initiation factor 3 subunit G"
}